{
  "term_id": "GO:2000391",
  "term_label": "positive regulation of neutrophil extravasation",
  "gene_name": "Glycoprotein Xg",
  "gene_symbol": "XG",
  "gene": "UniProtKB:P55808"
}